phosphatidylcholine floppase activity [GO:0090554] (molecular function) Definition: Catalysis of the movement of phosphatidylcholine from the cytosolic to the exoplasmic leaflet of a membrane, using energy from the hydrolysis of ATP. Relationships: is a type of phosphatidylcholine transporter activity [GO:0008525]; is a type of floppase activity [GO:0140328] Also known as: ATP-dependent phosphatidylcholine transporter activity, ATPase-coupled phosphatidylcholine transporter activity, phosphatidylcholine-translocating ATPase activity, phosphatidylcholine floppase activity (cytosolic to exoplasmic leaflet) References: PMID:16452632 Sources: GOC:ab, RHEA:38583